UDP-N-acetylglucosamine 6-dehydrogenase activity [GO:0047004] (molecular function) Definition: Catalysis of the reaction: H2O + 2 NAD+ + UDP-N-acetyl-alpha-D-glucosamine = 3 H+ + 2 NADH + UDP-N-acetyl-2-amino-2-deoxy-D-glucuronate. Sources: EC:1.1.1.136, RHEA:13325 Also known as: UDP-2-acetamido-2-deoxy-D-glucose:NAD oxidoreductase activity, UDP-GLcNAc dehydrogenase activity, UDP-N-acetyl-D-glucosamine:NAD+ 6-oxidoreductase activity, UDPacetylglucosamine dehydrogenase activity, uridine diphosphoacetylglucosamine dehydrogenase activity Relationships: is a type of GO:0016616